{
  "gene_symbol": "LSR",
  "gene": "UniProtKB:Q86X29",
  "gene_name": "Lipolysis-stimulated lipoprotein receptor",
  "term_id": "GO:0005886",
  "term_label": "plasma membrane"
}